{
  "gene_symbol": "SLC25A46",
  "term_label": "mitochondrial fission",
  "gene_name": "Mitochondrial outer membrane protein SLC25A46",
  "gene": "UniProtKB:Q96AG3",
  "term_id": "GO:0000266"
}